{
  "term_id": "UNKNOWN:0002",
  "term_label": "Unknown biological process",
  "gene": "UniProtKB:Q9H579",
  "gene_name": "Protein MROH8",
  "gene_symbol": "MROH8"
}